{
  "term_id": "GO:0000978",
  "gene": "UniProtKB:Q9NP62",
  "term_label": "RNA polymerase II cis-regulatory region sequence-specific DNA binding",
  "gene_name": "Chorion-specific transcription factor GCMa",
  "gene_symbol": "GCM1"
}